{
  "gene": "UniProtKB:Q9NYW1",
  "term_label": "bitter taste receptor activity",
  "term_id": "GO:0033038",
  "gene_name": "Taste receptor type 2 member 9",
  "gene_symbol": "TAS2R9"
}